negative regulation of cellodextrin catabolic process [GO:2000928] (biological process) Sources: GOC:mengo_curators Definition: Any process that stops, prevents or reduces the frequency, rate or extent of cellodextrin catabolic process. Relationships: is_a GO:0009895; is a type of negative regulation of macromolecule metabolic process [GO:0010605]; is a type of negative regulation of carbohydrate metabolic process [GO:0045912]; is a type of regulation of cellodextrin catabolic process [GO:2000927]; negatively regulates cellodextrin catabolic process [GO:2000890] Also known as: negative regulation of cellodextrin catabolism